{
  "term_label": "sensory perception of sound",
  "gene_symbol": "MYO7A",
  "gene_name": "Unconventional myosin-VIIa",
  "term_id": "GO:0007605",
  "gene": "UniProtKB:Q13402"
}